{
  "gene_name": "Metalloproteinase inhibitor 1",
  "gene_symbol": "TIMP1",
  "term_id": "GO:0051045",
  "gene": "UniProtKB:P01033",
  "term_label": "negative regulation of membrane protein ectodomain proteolysis"
}